{
  "term_label": "catalytic step 2 spliceosome",
  "gene_name": "Heterogeneous nuclear ribonucleoprotein A1-like 3",
  "gene_symbol": "HNRNPA1L3",
  "term_id": "GO:0071013",
  "gene": "UniProtKB:A0A2R8Y4L2"
}